neutral lipid catabolic process [GO:0046461] (biological process) Relationships: is a type of GO:0006638 Subtypes: GO:0046464 Also known as: neutral lipid breakdown, neutral lipid catabolism, neutral lipid degradation Definition: The chemical reactions and pathways resulting in the breakdown of neutral lipids, lipids only soluble in solvents of very low polarity. Sources: GOC:ai